{
  "term_label": "double-stranded RNA binding",
  "gene_symbol": "STAU2",
  "gene": "UniProtKB:Q9NUL3",
  "gene_name": "Double-stranded RNA-binding protein Staufen homolog 2",
  "term_id": "GO:0003725"
}